{
  "gene": "UniProtKB:Q03014",
  "gene_name": "Hematopoietically-expressed homeobox protein HHEX",
  "gene_symbol": "HHEX",
  "term_label": "RNA polymerase II cis-regulatory region sequence-specific DNA binding",
  "term_id": "GO:0000978"
}